methanofuran biosynthetic process [GO:2001120] (biological process) Definition: The chemical reactions and pathways resulting in the formation of a methanofuran. Sources: GOC:mengo_curators Also known as: methanofuran biosynthesis Relationships: is a type of biosynthetic process [GO:0009058]; is a type of GO:2001119 Regulation: RO_0002211 by GO:1900351; negatively regulated by negative regulation of methanofuran biosynthetic process [GO:1900352]; positively regulated by positive regulation of methanofuran biosynthetic process [GO:1900353]